2-hydroxyhexa-2,4-dienoate hydratase activity [GO:0034856] (molecular function) Sources: UM-BBD_reactionID:r1281 Relationships: is a type of hydro-lyase activity [GO:0016836] Definition: Catalysis of the reaction: (2E,4E)-2-hydroxyhexa-2,4-dienoate + H2O = 4-hydroxy-2-oxohexanoate.